phenyloplast [GO:0062116] (cellular component) Relationships: is a type of plastid [GO:0009536] References: PMID:24683183 Definition: A chloroplast-derived plastid in which the solid form of phenol is stored.